{
  "gene_name": "Putative uncharacterized protein encoded by LINC00471",
  "gene": "UniProtKB:Q8N535",
  "gene_symbol": "LINC00471",
  "term_id": "UNKNOWN:0002",
  "term_label": "Unknown biological process"
}